{
  "term_label": "U1 snRNP",
  "gene_name": "U2 small nuclear ribonucleoprotein B''",
  "gene_symbol": "SNRPB2",
  "term_id": "GO:0005685",
  "gene": "UniProtKB:P08579"
}